{
  "gene_name": "Methyl-CpG-binding domain protein 3",
  "term_label": "negative regulation of transcription by RNA polymerase II",
  "gene_symbol": "MBD3",
  "gene": "UniProtKB:O95983",
  "term_id": "GO:0000122"
}